{
  "term_id": "GO:0030628",
  "gene": "UniProtKB:P26368",
  "gene_symbol": "U2AF2",
  "gene_name": "Splicing factor U2AF 65 kDa subunit",
  "term_label": "pre-mRNA 3'-splice site binding"
}